{
  "term_label": "GTPase activator activity",
  "gene_symbol": "ARHGAP30",
  "term_id": "GO:0005096",
  "gene_name": "Rho GTPase-activating protein 30",
  "gene": "UniProtKB:Q7Z6I6"
}